{
  "gene_name": "Retinitis pigmentosa 1-like 1 protein",
  "gene_symbol": "RP1L1",
  "term_label": "axoneme assembly",
  "gene": "UniProtKB:Q8IWN7",
  "term_id": "GO:0035082"
}